{
  "gene_name": "Alpha-crystallin B chain",
  "term_id": "GO:0009408",
  "term_label": "response to heat",
  "gene_symbol": "CRYAB",
  "gene": "UniProtKB:P02511"
}